{
  "term_id": "GO:0001508",
  "gene_symbol": "KCNV1",
  "term_label": "action potential",
  "gene": "UniProtKB:Q6PIU1",
  "gene_name": "Potassium voltage-gated channel subfamily V member 1"
}